{
  "gene_name": "Golgi SNAP receptor complex member 1",
  "gene": "UniProtKB:O95249",
  "term_label": "endoplasmic reticulum to Golgi vesicle-mediated transport",
  "gene_symbol": "GOSR1",
  "term_id": "GO:0006888"
}